trace-amine receptor activity [GO:0001594] (molecular function) Relationships: is_a G protein-coupled amine receptor activity [GO:0008227] References: PMID:19325074 Sources: GOC:mah Subtypes: trimethylamine receptor activity [GO:1990081] Definition: Combining with a trace amine to initiate a change in cell activity. Trace amines are biogenic amines that are synthesized from aromatic amino acids and are substrates for monoamine oxidase, and are therefore detectable only at trace levels in mammals.